{
  "gene": "UniProtKB:P07737",
  "gene_name": "Profilin-1",
  "term_label": "regulation of actin filament polymerization",
  "gene_symbol": "PFN1",
  "term_id": "GO:0030833"
}